soyasaponin III rhamnosyltransferase activity [GO:0102241] (molecular function) Sources: EC:2.4.1.273, GOC:pz Definition: Catalysis of the reaction: UDP-L-rhamnose + soyasaponin III = H+ + UDP + soyasaponin I. Relationships: is a type of hexosyltransferase activity [GO:0016758]